indoleacetic acid catabolic process [GO:0042437] (biological process) Sources: GOC:jl Relationships: is a type of auxin catabolic process [GO:0009852]; is a type of indole-containing compound catabolic process [GO:0042436]; is a type of monocarboxylic acid catabolic process [GO:0072329] Also known as: IAA catabolic process, indole acetic acid catabolic process, indole acetic acid catabolism, indoleacetic acid breakdown, indoleacetic acid catabolism, indoleacetic acid degradation Definition: The chemical reactions and pathways resulting in the breakdown of indole-3-acetic acid, a compound which functions as a growth regulator in plants.